{
  "term_label": "protein kinase binding",
  "gene": "UniProtKB:Q6S8J3",
  "gene_symbol": "POTEE",
  "gene_name": "POTE ankyrin domain family member E",
  "term_id": "GO:0019901"
}